{
  "gene": "UniProtKB:Q13477",
  "term_label": "leukocyte tethering or rolling",
  "gene_name": "Mucosal addressin cell adhesion molecule 1",
  "gene_symbol": "MADCAM1",
  "term_id": "GO:0050901"
}